{
  "gene": "UniProtKB:Q15759",
  "term_label": "cytoplasm",
  "term_id": "GO:0005737",
  "gene_name": "Mitogen-activated protein kinase 11",
  "gene_symbol": "MAPK11"
}